{
  "gene": "UniProtKB:P10398",
  "term_id": "GO:0005739",
  "term_label": "mitochondrion",
  "gene_name": "Serine_threonine-protein kinase A-Raf",
  "gene_symbol": "ARAF"
}